{
  "gene_symbol": "OR4M2",
  "term_label": "plasma membrane",
  "term_id": "GO:0005886",
  "gene": "UniProtKB:Q8NGB6",
  "gene_name": "Olfactory receptor 4M2"
}